{
  "gene": "UniProtKB:Q9H1D9",
  "term_label": "Unknown molecular function",
  "gene_name": "DNA-directed RNA polymerase III subunit RPC6",
  "term_id": "UNKNOWN:0001",
  "gene_symbol": "POLR3F"
}